{
  "term_label": "plasma membrane",
  "gene": "UniProtKB:Q9H228",
  "gene_symbol": "S1PR5",
  "term_id": "GO:0005886",
  "gene_name": "Sphingosine 1-phosphate receptor 5"
}